{
  "term_label": "ribosomal small subunit binding",
  "term_id": "GO:0043024",
  "gene_name": "ATP-binding cassette sub-family E member 1",
  "gene_symbol": "ABCE1",
  "gene": "UniProtKB:P61221"
}